{
  "term_label": "regulation of DNA damage response, signal transduction by p53 class mediator",
  "gene_name": "N-lysine methyltransferase KMT5A",
  "gene": "UniProtKB:Q9NQR1",
  "gene_symbol": "KMT5A",
  "term_id": "GO:0043516"
}